fructose biosynthetic process [GO:0046370] (biological process) Definition: The chemical reactions and pathways resulting in the formation of fructose, the ketohexose arabino-2-hexulose. Relationships: is a type of GO:0006000; is a type of hexose biosynthetic process [GO:0019319] Also known as: fructose anabolism, fructose biosynthesis, fructose formation, fructose synthesis Sources: GOC:ai